{
  "gene_symbol": "POC5",
  "gene": "UniProtKB:Q8NA72",
  "term_label": "photoreceptor connecting cilium",
  "term_id": "GO:0032391",
  "gene_name": "Centrosomal protein POC5"
}